{
  "term_id": "GO:0003725",
  "gene": "UniProtKB:Q9NS39",
  "term_label": "double-stranded RNA binding",
  "gene_name": "Double-stranded RNA-specific editase B2",
  "gene_symbol": "ADARB2"
}